{
  "term_label": "cytoplasm",
  "gene_symbol": "LYPLA2",
  "gene_name": "Acyl-protein thioesterase 2",
  "gene": "UniProtKB:O95372",
  "term_id": "GO:0005737"
}